{
  "gene_symbol": "CNFN",
  "term_id": "GO:0001533",
  "term_label": "cornified envelope",
  "gene_name": "Cornifelin",
  "gene": "UniProtKB:Q9BYD5"
}